{
  "gene_symbol": "ABTB2",
  "gene": "UniProtKB:Q8N961",
  "gene_name": "Ankyrin repeat and BTB_POZ domain-containing protein 2",
  "term_label": "Unknown biological process",
  "term_id": "UNKNOWN:0002"
}